{
  "gene_symbol": "TRBJ1-2",
  "term_label": "Unknown molecular function",
  "gene": "UniProtKB:A0A0J9YX06",
  "term_id": "UNKNOWN:0001",
  "gene_name": "T cell receptor beta joining 1-2"
}